vascular endothelial growth factor receptor activity [GO:0005021] (molecular function) Definition: Combining with a vascular endothelial growth factor (VEGF) receptor ligand and transmitting the signal across the plasma membrane to initiate a change in cell activity. Also known as: VEGF receptor activity, VEGF-activated receptor activity, VEGFR activity, vascular endothelial growth factor E-activated receptor activity, vascular endothelial growth factor-activated receptor activity, VEGF-A-activated receptor activity, VEGF-B-activated receptor activity, VEGF-C-activated receptor activity, VEGF-D-activated receptor activity, VEGF-E-activated receptor activity Relationships: is_a GO:0004714; is part of GO:0038084; has part vascular endothelial growth factor binding [GO:0038085] References: PMID:19909239 Sources: GOC:mah, GOC:signaling Note: Note that this term represents an activity and not a gene product, and should only be used when the receptor binds the ligand VEGF. For receptors that bind other growth factors, consider annotating to terms under 'transmembrane signaling receptor activity ; GO:0004888.